{
  "term_id": "GO:0005739",
  "gene": "UniProtKB:Q15118",
  "term_label": "mitochondrion",
  "gene_symbol": "PDK1",
  "gene_name": "[Pyruvate dehydrogenase (acetyl-transferring)] kinase isozyme 1, mitochondrial"
}